{
  "term_label": "GTPase activator activity",
  "gene_name": "Arf-GAP with GTPase, ANK repeat and PH domain-containing protein 4",
  "gene": "UniProtKB:Q96P64",
  "term_id": "GO:0005096",
  "gene_symbol": "AGAP4"
}